GTP-dependent polynucleotide 5'-hydroxyl-kinase activity [GO:0051735] (molecular function) Definition: Catalysis of the reaction: GTP + 5'-dephosphopolynucleotide = GDP + 5'-phosphopolynucleotide. The polynucleotide may be DNA or RNA. Subtypes: GTP-dependent polyribonucleotide 5'-hydroxyl-kinase activity [GO:0051730], GTP-dependent polydeoxyribonucleotide 5'-hydroxyl-kinase activity [GO:0051737] Also known as: GTP-dependent polynucleotide kinase activity Sources: GOC:curators Relationships: is a type of GO:0051731